positive regulation of single strand break repair [GO:1903518] (BP) Definition: Any process that activates or increases the frequency, rate or extent of single strand break repair. References: PMID:17395247 Sources: GOC:BHF, GOC:TermGenie, GOC:rl, GO_REF:0000058 Subtypes: positive regulation of single-strand break repair via homologous recombination [GO:1903112] Relationships: is a type of positive regulation of DNA repair [GO:0045739]; is a type of GO:1903516; positively regulates single strand break repair [GO:0000012] Also known as: up regulation of single strand break repair, up-regulation of single strand break repair, upregulation of single strand break repair, activation of single strand break repair